positive regulation of myeloid dendritic cell antigen processing and presentation [GO:0002609] (biological process) Sources: GOC:add Definition: Any process that activates or increases the frequency, rate, or extent of myeloid dendritic cell antigen processing and presentation. Also known as: up regulation of myeloid dendritic cell antigen processing and presentation, up-regulation of myeloid dendritic cell antigen processing and presentation, upregulation of myeloid dendritic cell antigen processing and presentation, activation of myeloid dendritic cell antigen processing and presentation, stimulation of myeloid dendritic cell antigen processing and presentation Relationships: is a type of positive regulation of dendritic cell antigen processing and presentation [GO:0002606]; is a type of regulation of myeloid dendritic cell antigen processing and presentation [GO:0002607]; positively regulates myeloid dendritic cell antigen processing and presentation [GO:0002469]